{
  "term_label": "protein phosphatase binding",
  "term_id": "GO:0019903",
  "gene_name": "C-type lectin domain family 12 member B",
  "gene": "UniProtKB:Q2HXU8",
  "gene_symbol": "CLEC12B"
}